{
  "term_id": "GO:0030672",
  "gene_symbol": "STX6",
  "gene_name": "Syntaxin-6",
  "term_label": "synaptic vesicle membrane",
  "gene": "UniProtKB:O43752"
}